{
  "gene_symbol": "MDFIC2",
  "term_label": "regulation of Wnt signaling pathway",
  "gene": "UniProtKB:A0A1B0GVS7",
  "gene_name": "MyoD family inhibitor domain-containing protein 2",
  "term_id": "GO:0030111"
}